{
  "gene": "UniProtKB:Q9NUL7",
  "term_id": "UNKNOWN:0001",
  "gene_symbol": "DDX28",
  "gene_name": "Probable ATP-dependent RNA helicase DDX28",
  "term_label": "Unknown molecular function"
}